epiboly [GO:0090504] (biological process) Sources: GOC:dph, GOC:tb Subtypes: epiboly involved in gastrulation with mouth forming second [GO:0055113], epiboly involved in wound healing [GO:0090505] Definition: The expansion of one cell sheet over other cells or yolk. Relationships: is a type of morphogenesis of an epithelial sheet [GO:0002011]